{
  "term_id": "GO:0097745",
  "gene_name": "tRNA methyltransferase 10 homolog C",
  "gene": "UniProtKB:Q7L0Y3",
  "term_label": "mitochondrial tRNA 5'-end processing",
  "gene_symbol": "TRMT10C"
}